{
  "term_id": "GO:0000977",
  "gene": "UniProtKB:O60682",
  "gene_name": "Musculin",
  "term_label": "RNA polymerase II transcription regulatory region sequence-specific DNA binding",
  "gene_symbol": "MSC"
}